Edg-1 sphingosine 1-phosphate receptor binding [GO:0031754] (molecular function) Also known as: Edg-1 sphingosine 1-phosphate receptor ligand Definition: Binding to an Edg-1 sphingosine 1-phosphate receptor. Sources: GOC:mah, GOC:nln Relationships: is a type of endothelial differentiation G protein-coupled receptor binding [GO:0031753]